{
  "gene": "UniProtKB:Q6RI45",
  "term_id": "GO:0007010",
  "gene_symbol": "BRWD3",
  "gene_name": "Bromodomain and WD repeat-containing protein 3",
  "term_label": "cytoskeleton organization"
}